{
  "term_label": "chemical synaptic transmission",
  "gene_symbol": "PENK",
  "term_id": "GO:0007268",
  "gene_name": "Proenkephalin-A",
  "gene": "UniProtKB:P01210"
}